{
  "term_id": "GO:0097227",
  "gene_symbol": "SEPTIN4",
  "term_label": "sperm annulus",
  "gene_name": "Septin-4",
  "gene": "UniProtKB:O43236"
}